{
  "gene_symbol": "IL17D",
  "gene": "UniProtKB:Q8TAD2",
  "term_label": "cytokine activity",
  "gene_name": "Interleukin-17D",
  "term_id": "GO:0005125"
}